detection of mechanical stimulus involved in equilibrioception [GO:0050973] (biological process) Also known as: equilibrioception, detection of mechanical stimulus, equilibrioception, sensory detection of mechanical stimulus, equilibrioception, sensory transduction of mechanical stimulus, sensory detection of mechanical stimulus during equilibrioception, sensory transduction of mechanical stimulus during equilibrioception Sources: GOC:ai, GOC:dos Definition: The series of events involved in equilibrioception in which a mechanical stimulus is received and converted into a molecular signal. During equilibrioception, mechanical stimuli may be in the form of input from pressure receptors or from the labyrinth system of the inner ears. Relationships: is a type of GO:0050974; is part of equilibrioception [GO:0050957]